tRNA (m2G10) methyltransferase complex [GO:0043528] (cellular component) Definition: A protein complex required for the methylation of the guanosine nucleotide at position 10 (m2G10) in tRNA. In S. cerevisiae, this complex consists of at least two subunits, Trm11p and Trm112p. Relationships: is a type of GO:0043527 References: PMID:15899842